vascular endothelial growth factor receptor-3 signaling pathway [GO:0036325] (biological process) Sources: GOC:bf, GOC:uh, Wikipedia:VEGFR3, Wikipedia:VEGF_receptors Relationships: is a type of vascular endothelial growth factor receptor signaling pathway [GO:0048010] Also known as: FLT4 signaling pathway, VEGFR-3 signaling pathway, VEGFR3 signaling pathway Definition: The series of molecular signals initiated by a ligand binding to a vascular endothelial growth factor receptor-3 (VEGFR-3) on the surface of a target cell, and ending with the regulation of a downstream cellular process, e.g. transcription.